{
  "gene": "UniProtKB:Q13515",
  "term_label": "cytoskeleton",
  "gene_symbol": "BFSP2",
  "term_id": "GO:0005856",
  "gene_name": "Phakinin"
}